agmatine deiminase activity [GO:0047632] (molecular function) Definition: Catalysis of the reaction: agmatine + H2O = N-carbamoylputrescine + NH3. Relationships: is a type of GO:0016813 Sources: EC:3.5.3.12, MetaCyc:AGMATINE-DEIMINASE-RXN Also known as: agmatine amidinohydrolase, agmatine iminohydrolase activity